{
  "term_id": "GO:0005886",
  "gene": "UniProtKB:P18627",
  "gene_name": "Lymphocyte activation gene 3 protein",
  "gene_symbol": "LAG3",
  "term_label": "plasma membrane"
}